{
  "term_id": "UNKNOWN:0003",
  "term_label": "Unknown cellular component",
  "gene_symbol": "IGHV3-7",
  "gene": "UniProtKB:P01780",
  "gene_name": "Immunoglobulin heavy variable 3-7"
}